{
  "gene_symbol": "IRAK3",
  "gene_name": "Interleukin-1 receptor-associated kinase 3",
  "term_label": "Toll signaling pathway",
  "gene": "UniProtKB:Q9Y616",
  "term_id": "GO:0008063"
}